{
  "gene_symbol": "CTSD",
  "term_id": "GO:0006508",
  "gene_name": "Cathepsin D",
  "term_label": "proteolysis",
  "gene": "UniProtKB:P07339"
}